{
  "gene_symbol": "ARHGAP35",
  "gene": "UniProtKB:Q9NRY4",
  "term_id": "GO:0007266",
  "term_label": "Rho protein signal transduction",
  "gene_name": "Rho GTPase-activating protein 35"
}